{
  "gene_name": "Heat shock 70 kDa protein 1B",
  "term_id": "GO:0005634",
  "gene": "UniProtKB:P0DMV9",
  "gene_symbol": "HSPA1B",
  "term_label": "nucleus"
}